{
  "term_id": "UNKNOWN:0003",
  "gene_symbol": "MORN1",
  "gene_name": "MORN repeat-containing protein 1",
  "term_label": "Unknown cellular component",
  "gene": "UniProtKB:Q5T089"
}